{
  "gene_symbol": "BCO1",
  "term_id": "GO:0010436",
  "gene": "UniProtKB:Q9HAY6",
  "gene_name": "Beta,beta-carotene 15,15'-dioxygenase",
  "term_label": "carotenoid dioxygenase activity"
}